{
  "term_id": "GO:0005737",
  "gene": "UniProtKB:Q8WUX2",
  "gene_symbol": "CHAC2",
  "gene_name": "Glutathione-specific gamma-glutamylcyclotransferase 2",
  "term_label": "cytoplasm"
}